{
  "term_id": "GO:0030246",
  "gene_symbol": "LGALS8",
  "term_label": "carbohydrate binding",
  "gene": "UniProtKB:O00214",
  "gene_name": "Galectin-8"
}